{
  "gene_name": "Protein FAM72A",
  "gene_symbol": "FAM72A",
  "gene": "UniProtKB:Q5TYM5",
  "term_id": "GO:0005829",
  "term_label": "cytosol"
}